negative regulation of sporangium development [GO:0075312] (biological process) Relationships: is a type of negative regulation of spore-bearing organ development [GO:0075262]; is a type of regulation of sporangium development [GO:0075310]; negatively regulates GO:0043582 Definition: Any process that stops, prevents, or reduces the frequency, rate or extent of sporangium development, a process that leads to the formation of sporangium, a single-celled or many-celled structure in which spores are produced, as in fungi, algae, mosses, and ferns, gymnosperms, angiosperms. Sources: GOC:pamgo_curators Subtypes: negative regulation of sporangium germination [GO:0075225], GO:0075324